{
  "gene_symbol": "KCNA4",
  "gene_name": "Potassium voltage-gated channel subfamily A member 4",
  "gene": "UniProtKB:P22459",
  "term_id": "GO:0071805",
  "term_label": "potassium ion transmembrane transport"
}